{
  "gene_symbol": "PDCD4",
  "gene_name": "Programmed cell death protein 4",
  "term_label": "Unknown biological process",
  "gene": "UniProtKB:Q53EL6",
  "term_id": "UNKNOWN:0002"
}